organellar chromatophore [GO:0070111] (cellular component) Definition: A bacteroid-containing symbiosome in which the bacterial component is a genetically highly reduced cyanobacterium that is photosynthetically active and incapable of an independent existence outside its host. The chromatophore functions as a photosynthetic organelle, and has been found and characterized in the amoeba Paulinella chromatophora. References: PMID:18356055 Sources: GOC:expert_mm Relationships: is a type of bacteroid-containing symbiosome [GO:0043660] Also known as: Paulinella-type chromatophore